{
  "term_label": "DNA-binding transcription factor activity",
  "gene_name": "Homeobox protein Hox-D9",
  "gene": "UniProtKB:P28356",
  "term_id": "GO:0003700",
  "gene_symbol": "HOXD9"
}